{
  "gene": "UniProtKB:P50461",
  "term_id": "GO:0008307",
  "term_label": "structural constituent of muscle",
  "gene_symbol": "CSRP3",
  "gene_name": "Cysteine and glycine-rich protein 3"
}